{
  "gene_name": "Zinc finger protein 736",
  "gene_symbol": "ZNF736",
  "term_id": "GO:0006355",
  "term_label": "regulation of DNA-templated transcription",
  "gene": "UniProtKB:B4DX44"
}